{
  "term_id": "GO:0007187",
  "term_label": "G protein-coupled receptor signaling pathway, coupled to cyclic nucleotide second messenger",
  "gene": "UniProtKB:P28223",
  "gene_symbol": "HTR2A",
  "gene_name": "5-hydroxytryptamine receptor 2A"
}